{
  "gene_symbol": "DCDC2B",
  "gene_name": "Doublecortin domain-containing protein 2B",
  "term_id": "GO:0005874",
  "gene": "UniProtKB:A2VCK2",
  "term_label": "microtubule"
}